{
  "gene_name": "Abscission_NoCut checkpoint regulator",
  "term_id": "GO:0005813",
  "term_label": "centrosome",
  "gene_symbol": "ZFYVE19",
  "gene": "UniProtKB:Q96K21"
}